regulation of root hair elongation [GO:1902890] (biological process) Subtypes: GO:1902891, GO:1902892 Definition: Any process that modulates the frequency, rate or extent of root hair elongation. Relationships: is a type of regulation of cell growth [GO:0001558]; is a type of regulation of developmental growth [GO:0048638]; regulates root hair elongation [GO:0048767] References: PMID:22329353 Sources: GOC:TermGenie, GOC:als, GO_REF:0000058